{
  "term_id": "GO:0003735",
  "gene_name": "Large ribosomal subunit protein mL66",
  "gene": "UniProtKB:Q9NVS2",
  "term_label": "structural constituent of ribosome",
  "gene_symbol": "MRPS18A"
}